{
  "term_label": "extracellular space",
  "gene_name": "Complement C1q tumor necrosis factor-related protein 8",
  "gene_symbol": "C1QTNF8",
  "term_id": "GO:0005615",
  "gene": "UniProtKB:P60827"
}